18-methylnonadec-1-ene metabolic process [GO:1900880] (biological process) Subtypes: 18-methylnonadec-1-ene biosynthetic process [GO:1900881] Sources: GOC:TermGenie, GOC:mengo_curators Also known as: 18-methylnonadec-1-ene metabolism Definition: The chemical reactions and pathways involving 18-methylnonadec-1-ene. Relationships: is a type of olefin metabolic process [GO:1900673]